{
  "term_id": "UNKNOWN:0001",
  "gene_symbol": "LEAP2",
  "gene_name": "Liver-expressed antimicrobial peptide 2",
  "gene": "UniProtKB:Q969E1",
  "term_label": "Unknown molecular function"
}